{
  "gene_name": "Mitotic-spindle organizing protein 2B",
  "gene_symbol": "MZT2B",
  "term_id": "GO:0005813",
  "gene": "UniProtKB:Q6NZ67",
  "term_label": "centrosome"
}